{
  "gene_name": "LLGL scribble cell polarity complex component 2",
  "gene_symbol": "LLGL2",
  "gene": "UniProtKB:Q6P1M3",
  "term_label": "GTPase activator activity",
  "term_id": "GO:0005096"
}